{
  "gene_symbol": "JAML",
  "term_id": "GO:0072672",
  "gene": "UniProtKB:Q86YT9",
  "term_label": "neutrophil extravasation",
  "gene_name": "Junctional adhesion molecule-like"
}